{
  "term_label": "Unknown biological process",
  "gene_symbol": "FAM98B",
  "gene": "UniProtKB:Q52LJ0",
  "gene_name": "Protein FAM98B",
  "term_id": "UNKNOWN:0002"
}